positive regulation of dense core granule biogenesis [GO:2000707] (biological process) Definition: Any process that activates or increases the frequency, rate or extent of dense core granule biogenesis. Relationships: is a type of positive regulation of cellular component biogenesis [GO:0044089]; is a type of regulation of dense core granule biogenesis [GO:2000705]; positively regulates GO:0061110 Sources: GOC:obol